{
  "gene_name": "Putative uncharacterized protein CLLU1-AS1",
  "gene_symbol": "CLLU1-AS1",
  "term_label": "Unknown cellular component",
  "gene": "UniProtKB:Q5K130",
  "term_id": "UNKNOWN:0003"
}